{
  "gene_name": "Pulmonary surfactant-associated protein D",
  "term_id": "UNKNOWN:0001",
  "gene": "UniProtKB:P35247",
  "term_label": "Unknown molecular function",
  "gene_symbol": "SFTPD"
}